vitelline membrane formation [GO:0030704] (biological process) Definition: Construction of the vitelline membrane portion of the egg shell, a rigid structure required to maintain the shape of the egg. Sources: ISBN:0879694238 Relationships: is a type of developmental process involved in reproduction [GO:0003006]; is a type of cellular component assembly involved in morphogenesis [GO:0010927]; is a type of egg coat formation [GO:0035803]; is a type of extracellular matrix assembly [GO:0085029] Subtypes: vitelline membrane formation involved in chorion-containing eggshell formation [GO:0007305]